{
  "gene_symbol": "TMEM134",
  "term_id": "UNKNOWN:0002",
  "term_label": "Unknown biological process",
  "gene": "UniProtKB:Q9H6X4",
  "gene_name": "Transmembrane protein 134"
}